{
  "term_id": "GO:0007596",
  "gene_symbol": "PRRG4",
  "gene_name": "Transmembrane gamma-carboxyglutamic acid protein 4",
  "term_label": "blood coagulation",
  "gene": "UniProtKB:Q9BZD6"
}